{
  "gene": "UniProtKB:O75840",
  "gene_name": "Krueppel-like factor 7",
  "gene_symbol": "KLF7",
  "term_id": "GO:0005634",
  "term_label": "nucleus"
}